{
  "term_id": "UNKNOWN:0002",
  "gene_name": "Interleukin-17B",
  "gene_symbol": "IL17B",
  "gene": "UniProtKB:Q9UHF5",
  "term_label": "Unknown biological process"
}